{
  "gene": "UniProtKB:Q9UM54",
  "term_id": "GO:0042472",
  "gene_name": "Unconventional myosin-VI",
  "gene_symbol": "MYO6",
  "term_label": "inner ear morphogenesis"
}